plant septum development [GO:1905328] (biological process) Relationships: is a type of GO:0048856 Definition: The process whose specific outcome is the progression of a septum over time, from its formation to the mature structure. Subtypes: ovary septum development [GO:0080126], fruit septum development [GO:0080127], anther septum development [GO:0080128] Also known as: dissepiment development References: PMID:4562349 Sources: GOC:TermGenie, GOC:tb, GO_REF:0000080